venom-mediated suppression of sensory perception of pain [GO:0044741] (biological process) Also known as: envenomation resulting in inhibition of sensory perception of pain in other organism, envenomation resulting in negative regulation of sensory perception of pain in another organism, envenomation resulting in negative regulation of sensory perception of pain in other organism References: PMID:23034652 Sources: GOC:fj, GOC:jl Relationships: is a type of GO:0140136 Definition: A process in which an organism inhibits or disrupts sensory perception of pain in another organism via the action of a venom.